NatB complex [GO:0031416] (cellular component) Also known as: N-terminal acetyltransferase B complex Relationships: is a type of N-terminal protein acetyltransferase complex [GO:0031414] Definition: A conserved complex that catalyzes the transfer of an acetyl group to the N-terminal residue of a protein acceptor molecule that has a Met-Glu, Met-Asp, Met-Asn, or Met-Met N-terminus. In Saccharomyces the complex includes Nat3p and Mdm20p. References: PMID:12890471